{
  "gene_name": "Interleukin-17 receptor A",
  "gene": "UniProtKB:Q96F46",
  "gene_symbol": "IL17RA",
  "term_id": "UNKNOWN:0003",
  "term_label": "Unknown cellular component"
}